{
  "gene": "UniProtKB:P29728",
  "term_label": "interleukin-27-mediated signaling pathway",
  "gene_name": "2'-5'-oligoadenylate synthase 2",
  "gene_symbol": "OAS2",
  "term_id": "GO:0070106"
}